{
  "term_label": "regulation of transcription by RNA polymerase II",
  "gene_name": "Forkhead box protein D1",
  "gene_symbol": "FOXD1",
  "gene": "UniProtKB:Q16676",
  "term_id": "GO:0006357"
}